{
  "term_label": "GTPase activity",
  "gene": "UniProtKB:P61106",
  "term_id": "GO:0003924",
  "gene_symbol": "RAB14",
  "gene_name": "Ras-related protein Rab-14"
}